{
  "term_label": "NLS-bearing protein import into nucleus",
  "term_id": "GO:0006607",
  "gene": "UniProtKB:O60684",
  "gene_symbol": "KPNA6",
  "gene_name": "Importin subunit alpha-7"
}